{
  "gene": "UniProtKB:Q96PS8",
  "gene_symbol": "AQP10",
  "term_label": "plasma membrane",
  "gene_name": "Aquaporin-10",
  "term_id": "GO:0005886"
}